{
  "term_id": "GO:0004984",
  "gene": "UniProtKB:Q8NGI4",
  "gene_symbol": "OR4D11",
  "term_label": "olfactory receptor activity",
  "gene_name": "Olfactory receptor 4D11"
}